lithocholate 6beta-hydroxylase activity [GO:0033777] (molecular function) Sources: EC:1.14.14.138, RHEA:18857 Definition: Catalysis of the reaction: H+ + lithocholate + NADPH + O2 = 6-beta-hydroxylithocholate + H2O + NADP+. Relationships: is a type of GO:0016709 Also known as: 6beta-hydroxylase activity, CYP3A10, cytochrome P450 3A10/lithocholic acid 6beta-hydroxylase activity, lithocholate 6beta-monooxygenase activity, lithocholate,NADPH:oxygen oxidoreductase (6beta-hydroxylating) activity